positive regulation of tyramine signaling pathway [GO:2000133] (biological process) Sources: GOC:mah Also known as: positive regulation of tyramine signalling pathway Definition: Any process that activates or increases the frequency, rate or extent of tyramine signaling pathway. Relationships: is a type of positive regulation of octopamine or tyramine signaling pathway [GO:2000127]; is a type of regulation of tyramine signaling pathway [GO:2000131]; positively regulates tyramine signaling pathway [GO:0071928]